siroheme biosynthetic process [GO:0019354] (biological process) Definition: The chemical reactions and pathways resulting in the formation of siroheme, a tetrahydroporphyrin with adjacent, reduced pyrrole rings. Relationships: is a type of heme biosynthetic process [GO:0006783] Also known as: sirohaem biosynthesis, sirohaem biosynthetic process, siroheme anabolism, siroheme biosynthesis, siroheme formation, siroheme synthesis, siroheme synthase activity Sources: ISBN:0198506732